{
  "gene_name": "Serine racemase",
  "gene": "UniProtKB:Q9GZT4",
  "term_id": "GO:0005737",
  "gene_symbol": "SRR",
  "term_label": "cytoplasm"
}